{
  "gene": "UniProtKB:Q9BSJ5",
  "term_label": "Unknown cellular component",
  "gene_name": "Uncharacterized protein C17orf80",
  "gene_symbol": "C17orf80",
  "term_id": "UNKNOWN:0003"
}